{
  "term_id": "UNKNOWN:0002",
  "term_label": "Unknown biological process",
  "gene_name": "GTPase IMAP family member 4",
  "gene": "UniProtKB:Q9NUV9",
  "gene_symbol": "GIMAP4"
}